{
  "gene_symbol": "SPATA46",
  "gene_name": "Spermatogenesis-associated protein 46",
  "term_id": "GO:0031965",
  "term_label": "nuclear membrane",
  "gene": "UniProtKB:Q5T0L3"
}